cranial ganglion structural organization [GO:0061562] (biological process) Relationships: is a type of ganglion structural organization [GO:0061555]; is part of cranial nerve structural organization [GO:0021604]; is part of cranial ganglion morphogenesis [GO:0061559] Definition: The process that contributes to creating the structural organization of a cranial ganglion. This process pertains to the physical shaping of a rudimentary structure. Sources: GOC:dph Also known as: cranial ganglia structural organization Subtypes: GO:0061563